{
  "term_id": "GO:0005769",
  "gene": "UniProtKB:Q9Y2H2",
  "gene_symbol": "INPP5F",
  "term_label": "early endosome",
  "gene_name": "Phosphatidylinositide phosphatase SAC2"
}